{
  "gene_symbol": "LCE2B",
  "term_id": "UNKNOWN:0001",
  "term_label": "Unknown molecular function",
  "gene_name": "Late cornified envelope protein 2B",
  "gene": "UniProtKB:O14633"
}